[pyruvate kinase]-phosphatase activity [GO:0050408] (molecular function) Definition: Catalysis of the reaction: [pyruvate kinase] phosphate + H2O = [pyruvate kinase] + phosphate. Sources: EC:3.1.3.49, MetaCyc:PYRUVATE-KINASE-PHOSPHATASE-RXN Relationships: is a type of phosphoprotein phosphatase activity [GO:0004721] Also known as: ATP:pyruvate 2-O-phosphotransferase-phosphate phosphohydrolase activity, pyruvate kinase phosphatase activity, pyruvate kinase-phosphatase activity